nipple morphogenesis [GO:0060658] (biological process) Relationships: is a type of anatomical structure morphogenesis [GO:0009653]; is part of mammary gland morphogenesis [GO:0060443]; is part of GO:0060618 Sources: GOC:dph Definition: The process in which the nipple is generated and organized.